{
  "gene_symbol": "CCDC8",
  "term_id": "GO:0000226",
  "gene_name": "Coiled-coil domain-containing protein 8",
  "term_label": "microtubule cytoskeleton organization",
  "gene": "UniProtKB:Q9H0W5"
}